{
  "term_label": "transcription regulator complex",
  "term_id": "GO:0005667",
  "gene_name": "SKI family transcriptional corepressor 1",
  "gene": "UniProtKB:P84550",
  "gene_symbol": "SKOR1"
}